{
  "gene": "UniProtKB:A0A075B6S9",
  "gene_symbol": "IGKV1-37",
  "term_id": "UNKNOWN:0001",
  "term_label": "Unknown molecular function",
  "gene_name": "Probable non-functional immunoglobulinn kappa variable 1-37"
}